interleukin-7 receptor binding [GO:0005139] (MF) Definition: Binding to an interleukin-7 receptor. Also known as: IL-7, interleukin-7 receptor ligand Sources: GOC:ai Relationships: is a type of cytokine receptor binding [GO:0005126]; is a type of growth factor receptor binding [GO:0070851]